{
  "gene_name": "Armadillo repeat-containing protein 8",
  "term_id": "GO:0034657",
  "gene": "UniProtKB:Q8IUR7",
  "term_label": "GID complex",
  "gene_symbol": "ARMC8"
}